{
  "gene": "UniProtKB:Q9H8G1",
  "gene_symbol": "ZNF430",
  "term_label": "Unknown cellular component",
  "gene_name": "Zinc finger protein 430",
  "term_id": "UNKNOWN:0003"
}